sulfur oxidation, ferric ion-dependent [GO:0019423] (biological process) Sources: MetaCyc:FESULFOX-PWY Also known as: sulphur oxidation, ferric ion-dependent Definition: A sulfur oxidation process that proceeds via the reaction catalyzed by sulfur:ferric ion oxidoreductase, and requires the presence of ferric ion (Fe3+). Relationships: is a type of sulfur oxidation [GO:0019417]